{
  "gene_name": "Aftiphilin",
  "term_id": "GO:0030121",
  "term_label": "AP-1 adaptor complex",
  "gene": "UniProtKB:Q6ULP2",
  "gene_symbol": "AFTPH"
}